{
  "term_id": "GO:0045252",
  "gene_symbol": "OGDH",
  "term_label": "oxoglutarate dehydrogenase complex",
  "gene": "UniProtKB:Q02218",
  "gene_name": "2-oxoglutarate dehydrogenase complex component E1"
}